{
  "gene_name": "Biogenesis of lysosome-related organelles complex 1 subunit 2",
  "gene_symbol": "BLOC1S2",
  "gene": "UniProtKB:Q6QNY1",
  "term_label": "gamma-tubulin binding",
  "term_id": "GO:0043015"
}